3alpha-hydroxy bile acid-CoA-ester 3-dehydrogenase activity [GO:0033792] (molecular function) Note: Note that this was originally described as bile acid 7-dehydroxylase (PubMed:3549693). In fact, the 7-dehydroxylation process is catalyzed by multiple enzymes. Relationships: is a type of oxidoreductase activity, acting on the CH-OH group of donors, NAD or NADP as acceptor [GO:0016616] References: PMID:23836456 Sources: RHEA:55380 Definition: Catalysis of the reactions: a 3alpha-hydroxy bile acid CoA + NAD+ = a 3-oxo bile acid CoA + H+ + NADH. Also known as: 7alpha-dehydroxylase activity, bile acid 7-dehydroxylase activity, bile-acid 7alpha-dehydroxylase activity, cholate 7alpha-dehydroxylase activity